all-trans retinol 3,4-desaturase activity [GO:0061896] (molecular function) Definition: Catalysis of the reaction: all-trans-retinol + 2 H+ + O2 + 2 reduced [adrenodoxin] = all-trans-3,4-didehydro retinol + 2 H2O + 2 oxidized [adrenodoxin]. References: PMID:27059013 Relationships: is_a oxidoreductase activity, acting on paired donors, with incorporation or reduction of molecular oxygen [GO:0016705]